{
  "gene_name": "Paired box protein Pax-8",
  "gene": "UniProtKB:Q06710",
  "term_label": "regulation of transcription by RNA polymerase II",
  "gene_symbol": "PAX8",
  "term_id": "GO:0006357"
}